{
  "term_id": "GO:0005819",
  "gene_name": "Katanin p60 ATPase-containing subunit A1",
  "gene": "UniProtKB:O75449",
  "term_label": "spindle",
  "gene_symbol": "KATNA1"
}